bacterial-type flagellum filament [GO:0009420] (cellular component) Definition: The long (approximately 20 nm), thin external structure of the bacterial-type flagellum, which acts as a propeller. References: PMID:10572114, PMID:12624192 Sources: GOC:cilia, GOC:mtg_sensu Also known as: flagellar filament, flagellin-based flagellum filament Relationships: is a type of cellular anatomical structure [GO:0110165]; BFO_0000050 GO:0009288